{
  "gene": "UniProtKB:A6NHQ2",
  "gene_symbol": "FBLL1",
  "term_label": "nucleolus",
  "gene_name": "rRNA_tRNA 2'-O-methyltransferase fibrillarin-like protein 1",
  "term_id": "GO:0005730"
}